{
  "term_label": "Unknown cellular component",
  "gene_symbol": "LDAF1",
  "gene": "UniProtKB:Q96B96",
  "gene_name": "Lipid droplet assembly factor 1",
  "term_id": "UNKNOWN:0003"
}